{
  "gene": "UniProtKB:I3L3R5",
  "gene_name": "Coiled-coil domain-containing glutamate-rich protein 2",
  "term_label": "Unknown molecular function",
  "term_id": "UNKNOWN:0001",
  "gene_symbol": "CCER2"
}